{
  "gene_name": "Large ribosomal subunit protein uL15m",
  "term_id": "UNKNOWN:0002",
  "gene_symbol": "MRPL15",
  "gene": "UniProtKB:Q9P015",
  "term_label": "Unknown biological process"
}